{
  "gene_symbol": "APOBEC3A",
  "term_label": "defense response to virus",
  "term_id": "GO:0051607",
  "gene": "UniProtKB:P31941",
  "gene_name": "DNA dC-dU-editing enzyme APOBEC-3A"
}